2'-deoxymugineic-acid 2'-dioxygenase activity [GO:0033760] (molecular function) Relationships: is a type of 2-oxoglutarate-dependent dioxygenase activity [GO:0016706] Also known as: 2'-deoxymugineic acid,2-oxoglutarate:oxygen oxidoreductase (2-hydroxylating) activity, IDS3 Sources: EC:1.14.11.24, RHEA:12200 Definition: Catalysis of the reaction: 2'-deoxymugineate + 2-oxoglutarate + O2 = CO2 + H+ + mugineate + succinate.